vegetative to reproductive phase transition of meristem [GO:0010228] (biological process) Relationships: is a type of GO:0003006; is part of post-embryonic development [GO:0009791]; is part of reproductive structure development [GO:0048608] Definition: The process involved in transforming a meristem that produces vegetative structures, such as leaves, into a meristem that produces reproductive structures, such as a flower or an inflorescence. Also known as: transition from vegetative to reproductive phase, floral evocation, flowering Sources: GOC:tb